{
  "gene": "UniProtKB:Q96PC3",
  "term_id": "UNKNOWN:0001",
  "gene_symbol": "AP1S3",
  "term_label": "Unknown molecular function",
  "gene_name": "AP-1 complex subunit sigma-3"
}